{
  "gene_name": "NADPH-dependent diflavin oxidoreductase 1",
  "term_label": "Unknown biological process",
  "term_id": "UNKNOWN:0002",
  "gene": "UniProtKB:Q9UHB4",
  "gene_symbol": "NDOR1"
}